T=31/pseudo31 icosahedral capsid [GO:0160172] (cellular component) Definition: The protein coat that surrounds the infective nucleic acid in some virus particles where the subunits (capsomeres) are arranged to form an icosahedron with T=31 or pseudo T=31 symmetry. Sources: VZ:7036 Relationships: is a type of icosahedral viral capsid [GO:0019030]